{
  "gene_name": "Testis-expressed protein 15",
  "gene_symbol": "TEX15",
  "gene": "UniProtKB:Q9BXT5",
  "term_id": "GO:0010569",
  "term_label": "regulation of double-strand break repair via homologous recombination"
}